{
  "gene_symbol": "TRMO",
  "gene_name": "tRNA (adenine(37)-N6)-methyltransferase",
  "term_label": "Unknown cellular component",
  "term_id": "UNKNOWN:0003",
  "gene": "UniProtKB:Q9BU70"
}